positive regulation of mitochondrial translation in response to stress [GO:0010892] (biological process) Definition: Any process that activates or increases the frequency, rate or extent of mitochondrial translation as a result of a stimulus indicating the organism is under stress. References: PMID:8830768 Sources: GOC:dph, GOC:jp, GOC:tb Relationships: is a type of GO:0032056; is a type of positive regulation of mitochondrial translation [GO:0070131]